sporulation resulting in formation of a cellular spore [GO:0030435] (biological process) Relationships: is a type of sporulation [GO:0043934]; is a type of anatomical structure formation involved in morphogenesis [GO:0048646] Regulation: regulated by regulation of sporulation resulting in formation of a cellular spore [GO:0042173]; negatively regulated by negative regulation of sporulation resulting in formation of a cellular spore [GO:0042174]; positively regulated by positive regulation of sporulation resulting in formation of a cellular spore [GO:0045881] Subtypes: sexual sporulation resulting in formation of a cellular spore [GO:0043935], asexual sporulation resulting in formation of a cellular spore [GO:0043936] Sources: GOC:mah, GOC:pamgo_curators, ISBN:0072992913 Note: Note that the synonym 'spore differentiation', like the term name and definition, refers to differentiation into a spore rather than any subsequent developmental changes that a spore may undergo. Definition: The process in which a relatively unspecialized cell acquires the specialized features of a cellular spore, a cell form that can be used for dissemination, for survival of adverse conditions because of its heat and desiccation resistance, and/or for reproduction. Also known as: cellular spore formation by sporulation, spore biosynthesis, spore differentiation, spore formation